{
  "gene": "UniProtKB:Q9Y5E5",
  "term_id": "GO:0007155",
  "gene_symbol": "PCDHB4",
  "term_label": "cell adhesion",
  "gene_name": "Protocadherin beta-4"
}